{
  "term_label": "Unknown cellular component",
  "term_id": "UNKNOWN:0003",
  "gene_symbol": "SMIM23",
  "gene": "UniProtKB:A6NLE4",
  "gene_name": "Small integral membrane protein 23"
}